cerebellar unipolar brush cell differentiation [GO:0021711] (biological process) Definition: The process in which neuroblasts acquire specialized structural and/or functional features that characterize the mature unipolar brush cell in the cerebellum. Differentiation includes the processes involved in commitment of a neuroblast to a unipolar brush cell fate. A unipolar brush cell is a glutamatergic interneuron found in the cerebellar cortex. Relationships: is a type of cell differentiation in hindbrain [GO:0021533]; is a type of central nervous system neuron differentiation [GO:0021953]; BFO_0000050 GO:0021684 References: PMID:15157725 Sources: GOC:cls, GOC:dgh, GOC:dph, GOC:jid, GO_REF:0000021